glycine betaine:proton symporter activity [GO:0015653] (molecular function) Also known as: glycine betaine:hydrogen symporter activity Sources: TC:2.A.15.1.1 Definition: Enables the transfer of a solute or solutes from one side of a membrane to the other according to the reaction: glycine betaine(out) + H+(out) = glycine betaine(in) + H+(in). Relationships: is a type of amino-acid betaine transmembrane transporter activity [GO:0015199]; is a type of quaternary ammonium group:proton symporter activity [GO:0015652]; is part of glycine betaine transport [GO:0031460]